{
  "gene": "UniProtKB:Q00536",
  "term_label": "synaptic vesicle",
  "gene_name": "Cyclin-dependent kinase 16",
  "gene_symbol": "CDK16",
  "term_id": "GO:0008021"
}